{
  "gene_name": "BCL2_adenovirus E1B 19 kDa protein-interacting protein 3",
  "gene_symbol": "BNIP3",
  "term_id": "UNKNOWN:0001",
  "term_label": "Unknown molecular function",
  "gene": "UniProtKB:Q12983"
}